negative regulation of beige fat cell differentiation [GO:0160276] (BP) Definition: Any process that stops, prevents or reduces the frequency, rate or extent of beige fat cell differentiation. References: PMID:35978186 Relationships: is_a negative regulation of fat cell differentiation [GO:0045599]; negatively regulates GO:0160274